{
  "gene": "UniProtKB:Q96MX6",
  "term_label": "Unknown biological process",
  "gene_symbol": "DNAAF10",
  "gene_name": "Dynein axonemal assembly factor 10",
  "term_id": "UNKNOWN:0002"
}